cytoplasmic vesicle [GO:0031410] (cellular component) Definition: A vesicle found in the cytoplasm of a cell. Sources: GOC:ai, GOC:mah, GOC:vesicles Also known as: cytoplasmic membrane bounded vesicle, cytoplasmic membrane-enclosed vesicle, cytoplasmic, membrane-bounded vesicle Relationships: is a type of intracellular vesicle [GO:0097708]; is part of cytoplasm [GO:0005737] Subtypes: GO:0000331, GO:0005768, Golgi-associated vesicle [GO:0005798], transport vesicle [GO:0030133], coated vesicle [GO:0030135], endocytic vesicle [GO:0030139], aleurone grain [GO:0033095], Cvt vesicle [GO:0033107], GO:0033117, GO:0033675, carotenoid vesicle [GO:0043702], GO:0044310, gut granule [GO:0044840], chitosome [GO:0045009], pigment granule [GO:0048770], chloroplast vesicle [GO:0062247], GO:0097487, synaptic vesicle protein transport vesicle [GO:0097547], sperm cytoplasmic droplet [GO:0097598], ciliary vesicle [GO:0097721], mitochondrion-derived vesicle [GO:0099073], GO:0099503, GO:0120002, granular vesicle [GO:1990005], amorphous vesicle [GO:1990006]